{
  "gene_name": "Synaptotagmin-1",
  "gene": "UniProtKB:P21579",
  "gene_symbol": "SYT1",
  "term_label": "calcium ion sensor activity",
  "term_id": "GO:0061891"
}